rubber cis-polyprenylcistransferase activity [GO:0050267] (molecular function) Relationships: is a type of prenyl diphosphate synthase activity [GO:0120531] Also known as: rubber transferase activity, cis-prenyl transferase activity, isopentenyl pyrophosphate cis-1,4-polyisoprenyl transferase activity, poly-cis-polyprenyl-diphosphate:isopentenyl-diphosphate polyprenylcistransferase activity, rubber allyltransferase activity, rubber polymerase activity, rubber prenyltransferase activity Definition: Catalysis of the reaction: (cis-prenyl)n-diphosphate + isopentenyl diphosphate = (cis-prenyl)(n+1)-diphosphate + diphosphate. Sources: RHEA:18801